{
  "gene": "UniProtKB:O00571",
  "term_id": "GO:0005634",
  "gene_name": "ATP-dependent RNA helicase DDX3X",
  "term_label": "nucleus",
  "gene_symbol": "DDX3X"
}